voltage-gated potassium channel activity involved in SA node cell action potential repolarization [GO:0086090] (molecular function) Relationships: is a type of voltage-gated potassium channel activity involved in cardiac muscle cell action potential repolarization [GO:0086008]; is part of membrane repolarization during SA node cell action potential [GO:0086052] Also known as: voltage-gated potassium channel activity involved in SAN cell action potential, voltage-gated potassium channel activity involved in sinoatrial node cell action potential, voltage-gated potassium channel activity involved in sinus node cell action potential Sources: GOC:BHF, GOC:mtg_cardiac_conduct_nov11 Definition: Enables the transmembrane transfer of a potassium ion by a voltage-gated channel through the plasma membrane of an SA node cell contributing to the repolarization phase of an action potential. A voltage-gated channel is a channel whose open state is dependent on the voltage across the membrane in which it is embedded.